eosinophil fate determination [GO:0035858] (biological process) Relationships: is_a GO:0001709; is part of eosinophil fate commitment [GO:0035854] Definition: The cell fate determination process in which a cell becomes capable of differentiating autonomously into an eosinophil cell regardless of its environment; upon determination, the cell fate cannot be reversed. Also known as: eosinophil cell fate determination Sources: CL:0000771, GOC:BHF, GOC:vk